{
  "term_id": "UNKNOWN:0003",
  "gene_symbol": "RTF1",
  "gene_name": "RNA polymerase-associated protein RTF1 homolog",
  "gene": "UniProtKB:Q92541",
  "term_label": "Unknown cellular component"
}